{
  "term_id": "UNKNOWN:0003",
  "gene": "UniProtKB:P0DP08",
  "term_label": "Unknown cellular component",
  "gene_symbol": "IGHV4-38-2",
  "gene_name": "Immunoglobulin heavy variable 4-38-2"
}